protein-DNA complex transport [GO:0015869] (biological process) Sources: GOC:ai Definition: The directed movement of protein-DNA complexes into, out of or within a cell, or between cells, by means of some agent such as a transporter or pore. Also known as: DNA-protein complex transport Relationships: is a type of GO:0006886; is a type of nucleobase-containing compound transport [GO:0015931]; is a type of protein-containing complex localization [GO:0031503]